sophorosyloxydocosanoate catabolic process [GO:0019436] (biological process) Definition: The chemical reactions and pathways resulting in the breakdown of sophorosyloxydocosanoate, 13-sophorosyloxydocosanoate 6',6''-diacetate. Sources: GOC:ai Relationships: is a type of GO:0019377 Also known as: sophorosyloxydocosanoate breakdown, sophorosyloxydocosanoate catabolism, sophorosyloxydocosanoate degradation